{
  "gene_name": "Immunoglobulin heavy variable 1_OR21-1 (non-functional) (Fragment)",
  "term_id": "GO:0003823",
  "gene": "UniProtKB:A0A087WYE8",
  "gene_symbol": "IGHV1OR21-1",
  "term_label": "antigen binding"
}